{
  "gene_name": "Potassium voltage-gated channel subfamily E member 2",
  "term_id": "GO:0044325",
  "term_label": "transmembrane transporter binding",
  "gene_symbol": "KCNE2",
  "gene": "UniProtKB:Q9Y6J6"
}